{
  "gene_name": "Coronin-1A",
  "gene_symbol": "CORO1A",
  "term_id": "GO:0016477",
  "term_label": "cell migration",
  "gene": "UniProtKB:P31146"
}